{
  "gene_name": "TATA-box-binding protein-associated factor 11-like protein 13",
  "term_label": "RNA polymerase II general transcription initiation factor activity",
  "term_id": "GO:0016251",
  "gene": "UniProtKB:A0A1W2PPH5",
  "gene_symbol": "TAF11L13"
}